{
  "term_label": "protein ubiquitination",
  "gene": "UniProtKB:Q96PM5",
  "gene_symbol": "RCHY1",
  "gene_name": "RING finger and CHY zinc finger domain-containing protein 1",
  "term_id": "GO:0016567"
}